{
  "gene": "UniProtKB:P09382",
  "term_id": "GO:0043236",
  "term_label": "laminin binding",
  "gene_symbol": "LGALS1",
  "gene_name": "Galectin-1"
}